{
  "gene_symbol": "PRPF8",
  "gene": "UniProtKB:Q6P2Q9",
  "gene_name": "Pre-mRNA-processing-splicing factor 8",
  "term_label": "U5 snRNP",
  "term_id": "GO:0005682"
}